{
  "gene_name": "Endogenous retrovirus group FC1 Env polyprotein",
  "gene": "UniProtKB:P60507",
  "term_id": "UNKNOWN:0001",
  "term_label": "Unknown molecular function",
  "gene_symbol": "ERVFC1"
}